{
  "gene": "UniProtKB:Q9HC84",
  "gene_symbol": "MUC5B",
  "term_label": "extracellular matrix structural constituent",
  "term_id": "GO:0005201",
  "gene_name": "Mucin-5B"
}